phospholipid biosynthetic process [GO:0008654] (biological process) Also known as: phospholipid anabolism, phospholipid biosynthesis, phospholipid formation, phospholipid synthesis Regulation: regulated by GO:0071071; negatively regulated by negative regulation of phospholipid biosynthetic process [GO:0071072]; positively regulated by positive regulation of phospholipid biosynthetic process [GO:0071073] Sources: ISBN:0198506732 Subtypes: GO:0006489, sphinganine-1-phosphate biosynthetic process [GO:0006669], sphingomyelin biosynthetic process [GO:0006686], GO:0009240, GO:0009245, GDP-alpha-D-mannosylchitobiosyldiphosphodolichol biosynthetic process [GO:0019347], geranyl diphosphate biosynthetic process [GO:0033384], geranylgeranyl diphosphate biosynthetic process [GO:0033386], phytyl diphosphate biosynthetic process [GO:0033521], Kdo2-lipid A biosynthetic process [GO:0036104], 4-amino-4-deoxy-alpha-L-arabinopyranosyl undecaprenyl phosphate biosynthetic process [GO:0036108], dolichyl monophosphate biosynthetic process [GO:0043048], GO:0045337, GO:0046474, GO:0050992, mannosyl-inositol phosphorylceramide biosynthetic process [GO:0051999], dolichol phosphate mannose biosynthetic process [GO:0180047], beta-L-Ara4N-lipid A biosynthetic process [GO:1901760], 5alpha,9alpha,10beta-labda-8(20),13-dien-15-yl diphosphate biosynthetic process [GO:1901949], copal-8-ol diphosphate(3-) biosynthetic process [GO:1902243], ceramide phosphoethanolamine biosynthetic process [GO:1905373] Definition: The chemical reactions and pathways resulting in the formation of a phospholipid, a lipid containing phosphoric acid as a mono- or diester. Relationships: is_a phospholipid metabolic process [GO:0006644]; is a type of lipid biosynthetic process [GO:0008610]; is a type of GO:0090407